{
  "gene": "UniProtKB:Q9NVH6",
  "term_label": "Unknown molecular function",
  "term_id": "UNKNOWN:0001",
  "gene_name": "Trimethyllysine dioxygenase, mitochondrial",
  "gene_symbol": "TMLHE"
}